iron ion transport [GO:0006826] (biological process) Sources: GOC:ai Subtypes: iron import into cell [GO:0033212], lactoferrin transport [GO:0033571], GO:0033572, iron ion transmembrane transport [GO:0034755], iron coordination entity transport [GO:1901678], xylem-to-phloem iron transport [GO:1990388] Definition: The directed movement of iron (Fe) ions into, out of or within a cell, or between cells, by means of some agent such as a transporter or pore. Regulation: regulated by GO:0034756; RO_0002212 by negative regulation of iron ion transport [GO:0034757]; positively regulated by positive regulation of iron ion transport [GO:0034758] Relationships: is a type of transition metal ion transport [GO:0000041] Also known as: iron transport, ferric ion import, ferric ion transport, ferric iron import, ferric iron transport, ferric iron uptake, ferrous ion transport, ferrous iron transport, iron ion import